{
  "gene": "UniProtKB:Q9NVH0",
  "gene_name": "Exonuclease 3'-5' domain-containing protein 2",
  "gene_symbol": "EXD2",
  "term_label": "Unknown biological process",
  "term_id": "UNKNOWN:0002"
}